{
  "gene_name": "Disintegrin and metalloproteinase domain-containing protein 20",
  "gene": "UniProtKB:O43506",
  "gene_symbol": "ADAM20",
  "term_label": "metalloendopeptidase activity",
  "term_id": "GO:0004222"
}